{
  "gene_name": "TGF-beta-activated kinase 1 and MAP3K7-binding protein 2",
  "term_label": "K63-linked polyubiquitin modification-dependent protein binding",
  "gene_symbol": "TAB2",
  "gene": "UniProtKB:Q9NYJ8",
  "term_id": "GO:0070530"
}